negative regulation of mesoderm development [GO:2000381] (biological process) Definition: Any process that stops, prevents or reduces the frequency, rate or extent of mesoderm development. Sources: GOC:BHF Relationships: is a type of negative regulation of developmental process [GO:0051093]; is a type of regulation of mesoderm development [GO:2000380]; negatively regulates GO:0007498 Subtypes: negative regulation of mesoderm formation [GO:1905903]